{
  "gene_symbol": "TDRD6",
  "gene_name": "Tudor domain-containing protein 6",
  "term_label": "P granule",
  "term_id": "GO:0043186",
  "gene": "UniProtKB:O60522"
}